{
  "term_id": "GO:0055056",
  "term_label": "D-glucose transmembrane transporter activity",
  "gene": "UniProtKB:P11166",
  "gene_symbol": "SLC2A1",
  "gene_name": "Solute carrier family 2, facilitated glucose transporter member 1"
}